{
  "gene_symbol": "PRKAR2B",
  "term_label": "protein kinase A catalytic subunit binding",
  "term_id": "GO:0034236",
  "gene_name": "cAMP-dependent protein kinase type II-beta regulatory subunit",
  "gene": "UniProtKB:P31323"
}